dihydropyrimidinase activity [GO:0004157] (molecular function) Relationships: is a type of GO:0016812 Also known as: 5,6-dihydropyrimidine amidohydrolase activity, D-hydantoinase activity, hydantoin peptidase activity, hydantoinase activity, hydropyrimidine hydrase activity, pyrimidine hydrase activity Sources: EC:3.5.2.2 Definition: Catalysis of the reaction: 5,6-dihydrouracil + H2O = 3-ureidopropionate.